{
  "term_label": "Ras protein signal transduction",
  "gene": "UniProtKB:Q8N431",
  "gene_symbol": "RASGEF1C",
  "term_id": "GO:0007265",
  "gene_name": "Ras-GEF domain-containing family member 1C"
}